{
  "gene_name": "Thioredoxin-like protein 4A",
  "gene": "UniProtKB:P83876",
  "gene_symbol": "TXNL4A",
  "term_id": "UNKNOWN:0002",
  "term_label": "Unknown biological process"
}